{
  "term_id": "GO:0008047",
  "gene": "UniProtKB:Q9NPA3",
  "gene_symbol": "MID1IP1",
  "term_label": "enzyme activator activity",
  "gene_name": "Mid1-interacting protein 1"
}